cibarial fish-trap bristle morphogenesis [GO:0048718] (biological process) Relationships: is a type of chaeta morphogenesis [GO:0008407]; is part of GO:0007453; BFO_0000050 GO:0048725 Sources: FBbt:00004136, GOC:rc Also known as: fish trap bristle morphogenesis Definition: The process in which the anatomical structures of a cibarial fish-trap bristle are generated and organized. A cibarial fish-trap bristle is a sensory bristle on the anterior plate of the cibarium.